positive regulation of establishment of endothelial barrier [GO:1903142] (biological process) Also known as: up regulation of establishment of endothelial barrier, up-regulation of establishment of endothelial barrier, upregulation of establishment of endothelial barrier, activation of establishment of endothelial barrier Relationships: is a type of positive regulation of endothelial cell development [GO:1901552]; is a type of GO:1903140; positively regulates establishment of endothelial barrier [GO:0061028] Definition: Any process that activates or increases the frequency, rate or extent of establishment of endothelial barrier. References: PMID:24851274 Sources: GOC:TermGenie, GOC:als, GO_REF:0000058